{
  "gene_name": "Gamma-aminobutyric acid receptor subunit delta",
  "term_id": "GO:1902711",
  "gene_symbol": "GABRD",
  "gene": "UniProtKB:O14764",
  "term_label": "GABA-A receptor complex"
}